{
  "term_label": "canonical Wnt signaling pathway",
  "gene": "UniProtKB:Q9H461",
  "term_id": "GO:0060070",
  "gene_symbol": "FZD8",
  "gene_name": "Frizzled-8"
}